regulation of potassium ion export across plasma membrane [GO:1903764] (biological process) Relationships: is a type of regulation of potassium ion transmembrane transport [GO:1901379]; RO_0002211 potassium ion export across plasma membrane [GO:0097623] Definition: Any process that modulates the frequency, rate or extent of potassium ion export across the plasma membrane. References: PMID:19646991 Sources: GOC:BHF, GOC:TermGenie, GOC:mtg_cardiac_conduct_nov11, GOC:rl, GO_REF:0000058 Also known as: regulation of potassium export, regulation of potassium export across plasma membrane, regulation of potassium ion export Subtypes: negative regulation of potassium ion export across plasma membrane [GO:1903765], positive regulation of potassium ion export across plasma membrane [GO:1903766]